plastid [GO:0009536] (cellular component) Subtypes: amyloplast [GO:0009501], GO:0009507, GO:0009509, etioplast [GO:0009513], leucoplast [GO:0009516], GO:0009537, cyanelle [GO:0009842], GO:0020011, gerontoplast [GO:0034400], GO:0062116 Definition: Any member of a family of organelles found in the cytoplasm of plants and some protists, which are membrane-bounded and contain DNA. Plant plastids develop from a common type, the proplastid. Relationships: is a type of intracellular membrane-bounded organelle [GO:0043231]; is part of cytoplasm [GO:0005737] Sources: GOC:jl, ISBN:0198547684